{
  "gene_symbol": "ZNF718",
  "term_label": "RNA polymerase II cis-regulatory region sequence-specific DNA binding",
  "gene_name": "Zinc finger protein 718",
  "term_id": "GO:0000978",
  "gene": "UniProtKB:Q3SXZ3"
}